ligamentous ossification [GO:0036076] (biological process) Relationships: is a type of GO:0001503 Sources: GO_REF:0000034 Definition: Ossification wherein bone tissue forms within ligamentous tissue. Note: Ligamentous ossification may occur via replacement ossification or metaplastic ossification or both in any one instance.